{
  "gene": "UniProtKB:Q8WTP8",
  "gene_symbol": "AEN",
  "term_label": "exonuclease activity",
  "term_id": "GO:0004527",
  "gene_name": "Apoptosis-enhancing nuclease"
}